{
  "gene": "UniProtKB:Q9BWH6",
  "term_label": "Unknown cellular component",
  "gene_symbol": "RPAP1",
  "gene_name": "RNA polymerase II-associated protein 1",
  "term_id": "UNKNOWN:0003"
}